{
  "term_id": "GO:0005739",
  "term_label": "mitochondrion",
  "gene_symbol": "MRRF",
  "gene": "UniProtKB:Q96E11",
  "gene_name": "Ribosome-recycling factor, mitochondrial"
}